telomere tethering at nuclear periphery [GO:0034398] (biological process) Relationships: is a type of telomere localization [GO:0034397] Sources: GOC:mah Subtypes: GO:0044820, meiotic telomere tethering at nuclear periphery [GO:0044821] Definition: The process in which a telomere is maintained in a specific location at the nuclear periphery.